Factor XII activation [GO:0002542] (biological process) Also known as: Hageman factor activation Definition: Any process that activates Factor XII (Hageman factor). Factor XII is a protein synthesized by the liver that circulates in an inactive form until it encounters collagen or basement membrane or activated platelets (as occurs at the site of endothelial injury). Factor XII then undergoes a conformational change (becoming factor XIIa), exposing an active serine center that can subsequently cleave protein substrates and activate a variety of mediator systems. Factor XII is a participant in the clotting cascade as well as the kinin cascade. Sources: GOC:jal, ISBN:0721601871 Relationships: is a type of GO:0002673; is a type of positive regulation of protein processing [GO:0010954]; is part of plasma kallikrein-kinin cascade [GO:0002353]; positively regulates activation of plasma proteins involved in acute inflammatory response [GO:0002541]